{
  "gene_name": "Protein FAM151B",
  "gene": "UniProtKB:Q6UXP7",
  "gene_symbol": "FAM151B",
  "term_id": "GO:0005615",
  "term_label": "extracellular space"
}